{
  "gene": "UniProtKB:Q12983",
  "term_label": "mitochondrial outer membrane permeabilization",
  "term_id": "GO:0097345",
  "gene_symbol": "BNIP3",
  "gene_name": "BCL2_adenovirus E1B 19 kDa protein-interacting protein 3"
}